{
  "gene": "UniProtKB:Q5T124",
  "term_id": "GO:0043161",
  "gene_name": "UBX domain-containing protein 11",
  "term_label": "proteasome-mediated ubiquitin-dependent protein catabolic process",
  "gene_symbol": "UBXN11"
}